{
  "gene_symbol": "ECSCR",
  "term_label": "negative regulation of angiogenesis",
  "gene_name": "Endothelial cell-specific chemotaxis regulator",
  "term_id": "GO:0016525",
  "gene": "UniProtKB:Q19T08"
}